regulation of lymphocyte apoptotic process [GO:0070228] (biological process) Sources: GOC:add, GOC:mtg_apoptosis, ISBN:0781765196 Note: Note that a lymphocyte is a cell of the B cell, T cell, or natural killer cell lineage (CL:0000542). Relationships: is_a GO:2000106; regulates lymphocyte apoptotic process [GO:0070227] Definition: Any process that modulates the occurrence or rate of lymphocyte death by apoptotic process. Subtypes: regulation of B cell apoptotic process [GO:0002902], negative regulation of lymphocyte apoptotic process [GO:0070229], positive regulation of lymphocyte apoptotic process [GO:0070230], GO:0070232, regulation of natural killer cell apoptotic process [GO:0070247] Also known as: regulation of lymphocyte apoptosis